{
  "term_id": "GO:0005634",
  "gene": "UniProtKB:Q8IUE0",
  "term_label": "nucleus",
  "gene_symbol": "TGIF2LY",
  "gene_name": "Homeobox protein TGIF2LY"
}